poly(A) binding [GO:0008143] (molecular function) Definition: Binding to a sequence of adenylyl residues in an RNA molecule, such as the poly(A) tail, a sequence of adenylyl residues at the 3' end of eukaryotic mRNA. Sources: GOC:jl Relationships: is a type of GO:0070717 Also known as: poly(A) binding, within an RNA molecule, poly(rA) binding, poly-A binding, polyadenylate binding